regulation of cytosolic calcium ion concentration [GO:0051480] (biological process) Relationships: is a type of intracellular calcium ion homeostasis [GO:0006874] Also known as: calcium ion homeostasis in cytoplasm, cytoplasmic calcium ion concentration regulation, cytoplasmic calcium ion homeostasis, regulation of calcium ion concentration in cytoplasm, regulation of cytoplasmic calcium ion concentration, calcium ion homeostasis in cytosol, cytosolic calcium ion concentration regulation, regulation of calcium ion concentration in cytosol Subtypes: circadian regulation of calcium ion oscillation [GO:0010617], GO:0099509, regulation of postsynaptic cytosolic calcium ion concentration [GO:0099566] Sources: GOC:ai, GOC:mah, GOC:rph Definition: Any process involved in the maintenance of an internal steady state of calcium ions within the cytosol of a cell or between the cytosol and its surroundings.